{
  "term_label": "ligand-gated monoatomic ion channel activity",
  "gene_name": "Glutamate receptor ionotropic, NMDA 1",
  "gene": "UniProtKB:Q05586",
  "term_id": "GO:0015276",
  "gene_symbol": "GRIN1"
}